{
  "term_id": "GO:0005654",
  "gene": "UniProtKB:Q15646",
  "gene_symbol": "OASL",
  "term_label": "nucleoplasm",
  "gene_name": "2'-5'-oligoadenylate synthase-like protein"
}